regulation of septum digestion after cytokinesis [GO:0010590] (biological process) Subtypes: GO:2001042, positive regulation of septum digestion after cytokinesis [GO:2001043] Relationships: is a type of GO:0050794; regulates GO:0000920 Definition: Any process that modulates the rate, frequency or extent of the process of physically separating the septal cell wall material by enzymatic digestion, that occurs after daughter cells are separated by cytokinesis. References: PMID:19959363, PMID:21246752, PMID:22786806 Sources: GOC:TermGenie, GOC:mtg_cell_cycle Also known as: regulation of mitotic cytokinetic cell separation, regulation of cell separation after cytokinesis, regulation of cell separation following cytokinesis